regulation of cardiac epithelial to mesenchymal transition [GO:0062042] (BP) Definition: Any process that modulates the rate, frequency or extent of cardiac epithelial to mesenchymal transition, a transition where a cardiac epithelial cell loses apical/basolateral polarity, severs intercellular adhesive junctions, degrades basement membrane components and becomes a migratory mesenchymal cell. References: PMID:20951801 Sources: GOC:BHF, GOC:rph Relationships: is a type of regulation of epithelial to mesenchymal transition [GO:0010717]; RO_0002211 cardiac epithelial to mesenchymal transition [GO:0060317] Subtypes: positive regulation of cardiac epithelial to mesenchymal transition [GO:0062043], negative regulation of cardiac epithelial to mesenchymal transition [GO:0062044], GO:0140049, regulation of epithelial to mesenchymal transition involved in endocardial cushion formation [GO:1905005]